positive regulation of response to cytokinesis checkpoint signaling [GO:1902148] (biological process) Relationships: is a type of positive regulation of response to cell cycle checkpoint signaling [GO:1902146]; is a type of regulation of response to cytokinesis checkpoint signaling [GO:1902147]; positively regulates response to cytokinesis checkpoint signaling [GO:0072399] Sources: GOC:TermGenie, GOC:mtg_cell_cycle Also known as: activation of cytokinesis checkpoint effector process, activation of response to signal involved in cytokinesis checkpoint, positive regulation of cytokinesis checkpoint effector process, positive regulation of response to signal involved in cytokinesis checkpoint, up regulation of cytokinesis checkpoint effector process, up regulation of response to cytokinesis checkpoint signaling, up regulation of response to signal involved in cytokinesis checkpoint, up-regulation of cytokinesis checkpoint effector process, up-regulation of response to cytokinesis checkpoint signaling, up-regulation of response to signal involved in cytokinesis checkpoint, upregulation of cytokinesis checkpoint effector process, upregulation of response to cytokinesis checkpoint signaling, upregulation of response to signal involved in cytokinesis checkpoint, activation of response to cytokinesis checkpoint signaling Definition: Any process that activates or increases the frequency, rate or extent of response to cytokinesis checkpoint signaling.